D-ribose biosynthetic process [GO:0019302] (biological process) Sources: ISBN:0198506732 Relationships: is a type of D-ribose metabolic process [GO:0006014]; is a type of pentose biosynthetic process [GO:0019322] Also known as: D-ribose anabolism, D-ribose biosynthesis, D-ribose formation, D-ribose synthesis Definition: The chemical reactions and pathways resulting in the formation of D-ribose, (ribo-pentose).